{
  "gene_name": "Homeobox protein GBX-2",
  "gene_symbol": "GBX2",
  "term_id": "GO:0000981",
  "gene": "UniProtKB:P52951",
  "term_label": "DNA-binding transcription factor activity, RNA polymerase II-specific"
}